{
  "gene_symbol": "E2F7",
  "term_label": "DNA-binding transcription factor activity, RNA polymerase II-specific",
  "gene": "UniProtKB:Q96AV8",
  "term_id": "GO:0000981",
  "gene_name": "Transcription factor E2F7"
}